antigen processing and presentation of endogenous peptide antigen via MHC class I via ER pathway, TAP-independent [GO:0002486] (biological process) Definition: The process in which an antigen-presenting cell expresses a peptide antigen of endogenous origin on its cell surface in association with an MHC class I protein complex following intracellular transport via a TAP-independent ER pathway. The peptide is typically a fragment of a larger endogenous protein which has been degraded within the cell and becomes associated with the MHC class I molecule in the ER following transport from the cytosol via a TAP-independent pathway. Class I here refers to classical class I molecules. Relationships: is a type of antigen processing and presentation of endogenous peptide antigen via MHC class I via ER pathway [GO:0002484] References: PMID:14647477, PMID:15771591 Sources: GOC:add Also known as: TAP-independent antigen processing and presentation of endogenous peptide antigen via MHC class I via ER pathway, TAP-independent endogenous peptide antigen processing and presentation via MHC class I via ER pathway, endogenous peptide antigen processing and presentation via MHC class I via ER pathway, TAP-independent